{
  "gene_symbol": "PIGZ",
  "gene_name": "GPI mannosyltransferase 4",
  "term_id": "GO:0006506",
  "term_label": "GPI anchor biosynthetic process",
  "gene": "UniProtKB:Q86VD9"
}